{
  "gene_name": "Tyrosyl-DNA phosphodiesterase 1",
  "term_id": "GO:0003690",
  "gene_symbol": "TDP1",
  "term_label": "double-stranded DNA binding",
  "gene": "UniProtKB:Q9NUW8"
}